{
  "term_label": "innate immune response",
  "gene_symbol": "BPIFA1",
  "term_id": "GO:0045087",
  "gene_name": "BPI fold-containing family A member 1",
  "gene": "UniProtKB:Q9NP55"
}